{
  "term_label": "Unknown molecular function",
  "gene_name": "Protein SSUH2 homolog",
  "gene": "UniProtKB:Q9Y2M2",
  "term_id": "UNKNOWN:0001",
  "gene_symbol": "SSUH2"
}